{
  "term_id": "GO:0005737",
  "gene": "UniProtKB:Q92918",
  "term_label": "cytoplasm",
  "gene_name": "Mitogen-activated protein kinase kinase kinase kinase 1",
  "gene_symbol": "MAP4K1"
}